{
  "term_id": "GO:0031593",
  "gene": "UniProtKB:Q8IYU4",
  "gene_symbol": "UBQLNL",
  "term_label": "polyubiquitin modification-dependent protein binding",
  "gene_name": "Ubiquilin-like protein"
}